fatty acid biosynthetic process [GO:0006633] (biological process) Definition: The chemical reactions and pathways resulting in the formation of a fatty acid, any of the aliphatic monocarboxylic acids that can be liberated by hydrolysis from naturally occurring fats and oils. Fatty acids are predominantly straight-chain acids of 4 to 24 carbon atoms, which may be saturated or unsaturated; branched fatty acids and hydroxy fatty acids also occur, and very long chain acids of over 30 carbons are found in waxes. Sources: GOC:mah, ISBN:0198506732 Subtypes: GO:0000954, unsaturated fatty acid biosynthetic process [GO:0006636], GO:0009107, fatty acid elongation [GO:0030497], long-chain fatty acid biosynthetic process [GO:0042759], very long-chain fatty acid biosynthetic process [GO:0042761], butyryl-CoA biosynthetic process [GO:0044578], short-chain fatty acid biosynthetic process [GO:0051790], medium-chain fatty acid biosynthetic process [GO:0051792], mycolic acid biosynthetic process [GO:0071768], methyl-branched fatty acid biosynthetic process [GO:1902321], monounsaturated fatty acid biosynthetic process [GO:1903966] Regulation: regulated by regulation of fatty acid biosynthetic process [GO:0042304]; negatively regulated by negative regulation of fatty acid biosynthetic process [GO:0045717]; positively regulated by positive regulation of fatty acid biosynthetic process [GO:0045723] Relationships: is a type of fatty acid metabolic process [GO:0006631]; is a type of lipid biosynthetic process [GO:0008610]; is a type of GO:0072330 Also known as: fatty acid anabolism, fatty acid biosynthesis, fatty acid formation, fatty acid synthesis